{
  "term_label": "ADP-ribosyl-[dinitrogen reductase] hydrolase activity",
  "gene_symbol": "OARD1",
  "gene_name": "ADP-ribose glycohydrolase OARD1",
  "term_id": "GO:0047407",
  "gene": "UniProtKB:Q9Y530"
}